{
  "gene": "UniProtKB:A6NI56",
  "term_id": "UNKNOWN:0003",
  "term_label": "Unknown cellular component",
  "gene_symbol": "CCDC154",
  "gene_name": "Coiled-coil domain-containing protein 154"
}